{
  "gene": "UniProtKB:Q9BWW4",
  "term_label": "nucleus",
  "gene_symbol": "SSBP3",
  "gene_name": "Single-stranded DNA-binding protein 3",
  "term_id": "GO:0005634"
}